{
  "term_id": "UNKNOWN:0002",
  "term_label": "Unknown biological process",
  "gene": "UniProtKB:A0A1W2PRE2",
  "gene_symbol": "A0A1W2PRE2",
  "gene_name": "Uncharacterized protein"
}